larval lymph gland hemocyte differentiation [GO:0035168] (biological process) References: PMID:14602069 Sources: GOC:bf, GOC:mtg_sensu Also known as: larval lymph gland arthropod blood cell differentiation Relationships: is a type of GO:0042386; is part of GO:0035167 Definition: The process in which a relatively unspecialized cell derived from the larval lymph gland acquires the specialized features of a mature hemocyte. The lymph gland consists of three to six bilaterally paired lobes that are attached to the cardioblasts during larval stages, and it degenerates during pupal stages. Hemocytes are blood cells associated with a hemocoel (the cavity containing most of the major organs of the arthropod body) which are involved in defense and clotting of hemolymph, but not involved in transport of oxygen. An example of this process is found in Drosophila melanogaster. Subtypes: lymph gland plasmatocyte differentiation [GO:0035169], GO:0035170, GO:0035171